{
  "term_id": "GO:0005737",
  "term_label": "cytoplasm",
  "gene_name": "Unconventional myosin-Ig",
  "gene_symbol": "MYO1G",
  "gene": "UniProtKB:B0I1T2"
}